response to DNA damage checkpoint signaling [GO:0072423] (BP) Definition: A process that occurs in response to signals generated as a result of DNA damage checkpoint signaling. Sources: GOC:mtg_cell_cycle Subtypes: response to G2 DNA damage checkpoint signaling [GO:0072426], response to intra-S DNA damage checkpoint signaling [GO:0072429], response to G1 DNA damage checkpoint signaling [GO:0072432] Regulation: regulated by GO:1902153; positively regulated by positive regulation of response to DNA damage checkpoint signaling [GO:1902154] Relationships: is a type of response to DNA integrity checkpoint signaling [GO:0072402] Also known as: DNA damage checkpoint effector process, response to signal involved in DNA damage checkpoint